fluconazole transmembrane transporter activity [GO:0015244] (molecular function) Definition: Enables the transfer of fluconazole from one side of a membrane to the other. Fluconazole is an antifungal drug used for oral candidiasis and cryptococcal meningitis; it is still under study for treatment of vaginal candidiasis and other fungal infections. Also known as: fluconazole transporter activity Sources: GOC:curators Subtypes: GO:0015313 Relationships: is a type of alcohol transmembrane transporter activity [GO:0015665]; is a type of GO:1901474; is part of GO:0015903